frizzled binding [GO:0005109] (molecular function) Definition: Binding to a frizzled (fz) receptor. Relationships: is a type of G protein-coupled receptor binding [GO:0001664] Sources: GOC:ceb Also known as: fz binding, frizzled ligand, frizzled-2 binding, frizzled-2 ligand, fz ligand, fz2 binding, fz2 ligand